glucose 1-dehydrogenase [NAD(P)+] activity [GO:0047936] (molecular function) Definition: Catalysis of the reaction: beta-D-glucose + NAD(P)+ = D-glucono-1,5-lactone + NAD(P)H. Note: This enzyme has similar activity with either NAD+ or NADP+. Sources: EC:1.1.1.47 Relationships: is a type of GO:0004344; is a type of oxidoreductase activity, acting on the CH-OH group of donors, NAD or NADP as acceptor [GO:0016616] Subtypes: GO:0047934, glucose 1-dehydrogenase (NADP+) activity [GO:0047935] Also known as: D-glucose dehydrogenase (NAD(P)), beta-D-glucose:NAD(P)+ 1-oxidoreductase activity, hexose phosphate dehydrogenase activity